{
  "gene": "UniProtKB:P00746",
  "gene_name": "Complement factor D",
  "term_label": "extracellular space",
  "gene_symbol": "CFD",
  "term_id": "GO:0005615"
}